{
  "term_label": "post-spliceosomal complex",
  "term_id": "GO:0071020",
  "gene_name": "Pre-mRNA-splicing factor ISY1 homolog",
  "gene_symbol": "ISY1",
  "gene": "UniProtKB:Q9ULR0"
}